RNA polymerase II C-terminal domain binding [GO:0099122] (molecular function) Relationships: is a type of RNA polymerase II complex binding [GO:0000993] Also known as: RNAP II C-terminal binding Subtypes: RNA polymerase II C-terminal domain phosphoserine binding [GO:1990269] References: PMID:20889714 Definition: Binding to the C-terminal domain (CTD) of the largest subunit of RNA polymerase II. The CTD is comprised of repeats of a heptapeptide with the consensus sequence YSPTSPS. The number of repeats varies with the species and a minimum number of repeats is required for RNAP II function.